{
  "term_label": "Unknown molecular function",
  "gene": "UniProtKB:Q5TGI0",
  "term_id": "UNKNOWN:0001",
  "gene_symbol": "FAXC",
  "gene_name": "Failed axon connections homolog"
}